{
  "term_id": "UNKNOWN:0001",
  "term_label": "Unknown molecular function",
  "gene_symbol": "ERVS71-1",
  "gene": "UniProtKB:P61550",
  "gene_name": "Endogenous retrovirus group S71 member 1 Env polyprotein"
}